{
  "term_id": "GO:0006865",
  "term_label": "amino acid transport",
  "gene_symbol": "SLC6A6",
  "gene": "UniProtKB:P31641",
  "gene_name": "Sodium- and chloride-dependent taurine transporter"
}